{
  "gene_symbol": "TMEM45B",
  "gene": "UniProtKB:Q96B21",
  "term_id": "UNKNOWN:0002",
  "term_label": "Unknown biological process",
  "gene_name": "Transmembrane protein 45B"
}